{
  "gene_symbol": "SFTPB",
  "gene_name": "Pulmonary surfactant-associated protein B",
  "term_label": "multivesicular body",
  "gene": "UniProtKB:P07988",
  "term_id": "GO:0005771"
}